mitotic spindle pole body insertion into the nuclear envelope [GO:0140480] (BP) Definition: A process in which the duplicated mitotic spindle pole body is inserted into a fenestra which opens in the nuclear envelope in early mitosis, and is subsequently tethered to the membrane. Also known as: establishment of spindle pole body localisation in nuclear envelope, establishment of spindle pole body localization in nuclear envelope, establishment of spindle pole body localization to nuclear envelope Relationships: is a type of GO:1990608 References: PMID:19487457, PMID:24529240